{
  "gene_symbol": "OLFML3",
  "gene_name": "Olfactomedin-like protein 3",
  "term_id": "GO:0005615",
  "term_label": "extracellular space",
  "gene": "UniProtKB:Q9NRN5"
}